{
  "gene_name": "CCR4-NOT transcription complex subunit 7",
  "term_id": "GO:0030015",
  "gene_symbol": "CNOT7",
  "term_label": "CCR4-NOT core complex",
  "gene": "UniProtKB:Q9UIV1"
}